{
  "term_label": "motile cilium",
  "gene_symbol": "ROPN1L",
  "gene_name": "Ropporin-1-like protein",
  "term_id": "GO:0031514",
  "gene": "UniProtKB:Q96C74"
}